{
  "gene": "UniProtKB:O75153",
  "gene_name": "Clustered mitochondria protein homolog",
  "term_id": "GO:0048312",
  "gene_symbol": "CLUH",
  "term_label": "intracellular distribution of mitochondria"
}